3,4-dihydroxybenzoate metabolic process [GO:0046278] (biological process) Relationships: is a type of GO:0009712; is a type of monocarboxylic acid metabolic process [GO:0032787]; is a type of benzene-containing compound metabolic process [GO:0042537] Also known as: protocatechuate metabolic process, protocatechuate metabolism References: PMID:24359411 Sources: GOC:ai Subtypes: 3,4-dihydroxybenzoate catabolic process [GO:0019619], 3,4-dihydroxybenzoate biosynthetic process [GO:0046279] Definition: The chemical reactions and pathways involving protocatechuate, the anion of protocatechuic acid (3,4-dihydroxybenzoic acid).